{
  "gene": "UniProtKB:P0CL84",
  "gene_name": "Putative STAG3-like protein 2",
  "term_label": "Unknown molecular function",
  "gene_symbol": "STAG3L2",
  "term_id": "UNKNOWN:0001"
}